positive regulation of pancreatic A cell differentiation [GO:2000228] (biological process) Sources: GOC:mah Definition: Any process that activates or increases the frequency, rate or extent of pancreatic A cell differentiation. Also known as: positive regulation of pancreatic alpha cell differentiation Relationships: is a type of positive regulation of epithelial cell differentiation [GO:0030858]; is a type of GO:0051240; is a type of GO:2000226; RO_0002213 pancreatic A cell differentiation [GO:0003310]